{
  "term_label": "Unknown cellular component",
  "gene": "UniProtKB:Q9Y5A7",
  "term_id": "UNKNOWN:0003",
  "gene_symbol": "NUB1",
  "gene_name": "NEDD8 ultimate buster 1"
}